{
  "term_id": "GO:0003700",
  "gene_name": "Heat shock factor protein 1",
  "gene_symbol": "HSF1",
  "term_label": "DNA-binding transcription factor activity",
  "gene": "UniProtKB:Q00613"
}